C-C motif chemokine 5 receptor activity [GO:0038122] (molecular function) Also known as: CCL5 receptor activity, RANTES receptor activity, small inducible cytokine A5 receptor activity Definition: Combining with the C-C motif chemokine 5 (CCL5) and transmitting the signal from one side of the membrane to the other to initiate a change in cell activity. Relationships: is a type of C-C chemokine receptor activity [GO:0016493]; is part of chemokine (C-C motif) ligand 5 signaling pathway [GO:0035689]; has part chemokine (C-C motif) ligand 5 binding [GO:0071791] Sources: GOC:signaling